{
  "gene_symbol": "CMPK2",
  "term_id": "GO:0006233",
  "term_label": "dTDP biosynthetic process",
  "gene_name": "UMP-CMP kinase 2, mitochondrial",
  "gene": "UniProtKB:Q5EBM0"
}